tripeptide transport [GO:0042939] (biological process) Subtypes: glutathione transport [GO:0034635], GO:0035443 Relationships: is a type of oligopeptide transport [GO:0006857] Sources: GOC:jl Definition: The directed movement of a tripeptide, a compound containing three amino acids linked together by peptide bonds, into, out of or within a cell, or between cells, by means of some agent such as a transporter or pore.